{
  "term_id": "GO:0012505",
  "gene_symbol": "STX1B",
  "term_label": "endomembrane system",
  "gene_name": "Syntaxin-1B",
  "gene": "UniProtKB:P61266"
}